protein localization to juxtaparanode region of axon [GO:0071205] (BP) Relationships: is a type of protein localization to axon [GO:0099612] Sources: GOC:BHF, GOC:mah Definition: Any process in which a protein is transported to, or maintained at, the juxtaparanode region of an axon. Also known as: protein localisation to juxtaparanode region of axon